positive regulation of cobalamin metabolic process [GO:0106121] (biological process) Definition: Any process that activates or increases the frequency, rate or extent of a cobalamin metabolic process. References: PMID:29056341 Relationships: is_a positive regulation of metabolic process [GO:0009893]; is a type of regulation of cobalamin metabolic process [GO:0106064]; positively regulates cobalamin metabolic process [GO:0009235]